Malpighian tubule stellate cell differentiation [GO:0061330] (biological process) Definition: The process in which a relatively unspecialized cell acquires specialized features of a Malpighian tubule stellate cell. A Malpighian tubule stellate cell is a specialized epithelial secretory cell that moves chloride ions and water across the tubule epithelium. References: PMID:19783135 Sources: GOC:dph, GOC:mtg_kidney_jan10 Relationships: is a type of epithelial cell differentiation [GO:0030855]; is part of Malpighian tubule development [GO:0072002]